{
  "gene": "UniProtKB:P40198",
  "gene_name": "Carcinoembryonic antigen-related cell adhesion molecule 3",
  "term_id": "GO:0007165",
  "term_label": "signal transduction",
  "gene_symbol": "CEACAM3"
}